{
  "gene": "UniProtKB:Q8N3J2",
  "gene_name": "N(6)-adenine-specific methyltransferase METTL4",
  "term_id": "GO:0009007",
  "gene_symbol": "METTL4",
  "term_label": "site-specific DNA-methyltransferase (adenine-specific) activity"
}